{
  "term_id": "GO:0005109",
  "gene_symbol": "NDP",
  "gene": "UniProtKB:Q00604",
  "gene_name": "Norrin",
  "term_label": "frizzled binding"
}